regulation of CD4-positive, alpha-beta T cell differentiation [GO:0043370] (biological process) Note: Note that immunologists typically use the word 'development' to refer to cells of B or T cell lineages undergoing the process that GO describes as 'cell differentiation'. Relationships: is a type of GO:0046637; is a type of regulation of CD4-positive, alpha-beta T cell activation [GO:2000514]; regulates GO:0043367 Definition: Any process that modulates the frequency, rate, or extent of CD4-positive, alpha-beta T cell differentiation. Subtypes: regulation of CD4-positive, CD25-positive, alpha-beta regulatory T cell differentiation [GO:0032829], negative regulation of CD4-positive, alpha-beta T cell differentiation [GO:0043371], positive regulation of CD4-positive, alpha-beta T cell differentiation [GO:0043372], regulation of T-helper cell differentiation [GO:0045622] Sources: GOC:add, GOC:pr, ISBN:0781735149 Also known as: regulation of CD4-positive T lymphocyte differentiation, regulation of CD4-positive T-cell differentiation, regulation of CD4-positive T-lymphocyte differentiation, regulation of CD4-positive, alpha beta T cell differentiation, regulation of CD4-positive, alpha beta T lymphocyte differentiation, regulation of CD4-positive, alpha beta T-cell differentiation, regulation of CD4-positive, alpha beta T-lymphocyte differentiation, regulation of CD4-positive, alpha beta T cell development